{
  "term_id": "GO:0001227",
  "gene_name": "Forkhead box protein P1",
  "gene": "UniProtKB:Q9H334",
  "term_label": "DNA-binding transcription repressor activity, RNA polymerase II-specific",
  "gene_symbol": "FOXP1"
}